{
  "gene_name": "Ephrin-A4",
  "gene": "UniProtKB:P52798",
  "term_id": "GO:0005886",
  "gene_symbol": "EFNA4",
  "term_label": "plasma membrane"
}